{
  "gene_symbol": "WDR53",
  "term_id": "UNKNOWN:0003",
  "gene": "UniProtKB:Q7Z5U6",
  "term_label": "Unknown cellular component",
  "gene_name": "WD repeat-containing protein 53"
}